{
  "gene_symbol": "IGHV3-20",
  "gene_name": "Immunoglobulin heavy variable 3-20",
  "gene": "UniProtKB:A0A0C4DH32",
  "term_id": "UNKNOWN:0003",
  "term_label": "Unknown cellular component"
}